positive regulation of ferrichrome biosynthetic process [GO:1905570] (biological process) Subtypes: GO:1900680 Definition: Any process that activates or increases the frequency, rate or extent of ferrichrome biosynthetic process. Relationships: is a type of positive regulation of amide metabolic process [GO:0034250]; is a type of positive regulation of siderophore biosynthetic process [GO:1900706]; is_a GO:1905568; positively regulates ferrichrome biosynthetic process [GO:0031169] Also known as: positive regulation of ferrichrome anabolism, positive regulation of ferrichrome biosynthesis, positive regulation of ferrichrome formation, positive regulation of ferrichrome synthesis, up regulation of ferrichrome anabolism, up regulation of ferrichrome biosynthesis, up regulation of ferrichrome biosynthetic process, up regulation of ferrichrome formation, up regulation of ferrichrome synthesis, up-regulation of ferrichrome anabolism, up-regulation of ferrichrome biosynthesis, up-regulation of ferrichrome biosynthetic process, up-regulation of ferrichrome formation, up-regulation of ferrichrome synthesis, upregulation of ferrichrome anabolism, upregulation of ferrichrome biosynthesis, upregulation of ferrichrome biosynthetic process, upregulation of ferrichrome formation, upregulation of ferrichrome synthesis, activation of ferrichrome anabolism, activation of ferrichrome biosynthesis, activation of ferrichrome biosynthetic process, activation of ferrichrome biosynthetic process, peptide formation, activation of ferrichrome biosynthetic process, peptide modification, activation of ferrichrome formation, activation of ferrichrome synthesis, positive regulation of ferrichrome biosynthetic process, peptide formation, positive regulation of ferrichrome biosynthetic process, peptide modification, up regulation of ferrichrome biosynthetic process, peptide formation, up regulation of ferrichrome biosynthetic process, peptide modification, up-regulation of ferrichrome biosynthetic process, peptide formation, up-regulation of ferrichrome biosynthetic process, peptide modification, upregulation of ferrichrome biosynthetic process, peptide formation, upregulation of ferrichrome biosynthetic process, peptide modification References: PMID:654321 Sources: GOC:TermGenie, GOC:al, GO_REF:0000058